{
  "gene_name": "Proepiregulin",
  "gene_symbol": "EREG",
  "term_label": "growth factor activity",
  "term_id": "GO:0008083",
  "gene": "UniProtKB:O14944"
}